{
  "gene_symbol": "FAM229B",
  "term_label": "Unknown cellular component",
  "gene": "UniProtKB:Q4G0N7",
  "term_id": "UNKNOWN:0003",
  "gene_name": "Protein FAM229B"
}